{
  "gene": "UniProtKB:Q7L7L0",
  "gene_symbol": "H2AC25",
  "term_id": "GO:0005634",
  "gene_name": "Histone H2A type 3",
  "term_label": "nucleus"
}